{
  "gene_name": "C-C motif chemokine 7",
  "term_id": "GO:0048245",
  "gene_symbol": "CCL7",
  "term_label": "eosinophil chemotaxis",
  "gene": "UniProtKB:P80098"
}